meiotic interphase II [GO:0044844] (biological process) Sources: GOC:jl, GOC:mtg_cell_cycle Relationships: is a type of meiotic interphase [GO:0051328]; is a type of meiosis II cell cycle phase [GO:0098765] Definition: The cell cycle phase which begins at the end of meiosis I cytokinesis and ends when meiosis II prophase begins. During meiotic interphase II no DNA replication takes place, but the centrioles duplicate and spindle fibres emerge. Note: Note that this term should not be used for direct annotation. If you are trying to make an annotation to x phase, it is likely that the correct annotation is 'regulation of x/y phase transition' or to a process which occurs during the reported phase (i.e mitotic DNA replication for mitotic S-phase). To capture the phase when a specific location or process is observed, the phase term can be used in an annotation extension (PMID:24885854) applied to a cellular component term (with the relation exists_during) or a biological process term (with the relation happens_during).